{
  "term_id": "UNKNOWN:0003",
  "gene_name": "Testis development-related protein 1",
  "term_label": "Unknown cellular component",
  "gene": "UniProtKB:Q3Y452",
  "gene_symbol": "TDRG1"
}